{
  "gene_symbol": "ZSCAN4",
  "gene_name": "Zinc finger and SCAN domain-containing protein 4",
  "term_id": "GO:0000981",
  "gene": "UniProtKB:Q8NAM6",
  "term_label": "DNA-binding transcription factor activity, RNA polymerase II-specific"
}